regulation of germ tube formation [GO:0075010] (biological process) Sources: GOC:pamgo_curators Relationships: is a type of regulation of developmental process [GO:0050793]; regulates germ tube formation [GO:0075009] Subtypes: positive regulation of germ tube formation [GO:0075011], negative regulation of germ tube formation [GO:0075012] Definition: Any process that modulates the frequency, rate or extent of germ tube formation on or near host. The host is defined as the larger of the organisms involved in a symbiotic interaction. Note: Note that this term should not be used to annotate gene products of the host. It should only be used to annotate those gene products from the symbiont involved in this process.